{
  "gene_name": "E3 ubiquitin-protein ligase UBR3",
  "gene_symbol": "UBR3",
  "gene": "UniProtKB:Q6ZT12",
  "term_id": "GO:0016567",
  "term_label": "protein ubiquitination"
}